diacyl lipopeptide binding [GO:0042498] (molecular function) Note: Note that bacterial lipopeptides are derived from bacterial lipoproteins, but the two terms are sometimes used interchangeably in the literature. Relationships: is a type of lipopeptide binding [GO:0071723] References: PMID:12077222, PMID:12524386, PMID:2757794 Sources: GOC:add Definition: Binding to a lipopeptide containing a nonprotein moiety consisting of two acyl groups. Also known as: diacylated lipopeptide binding, bacterial diacyl lipopeptide binding, bacterial diacyl lipoprotein binding